regulation of circadian sleep/wake cycle, REM sleep [GO:0042320] (biological process) References: PMID:11506998 Sources: GOC:jl Relationships: is a type of regulation of circadian sleep/wake cycle, sleep [GO:0045187]; regulates GO:0042747 Definition: Any process that modulates the frequency, rate or extent of rapid eye movement (REM) sleep. Subtypes: negative regulation of circadian sleep/wake cycle, REM sleep [GO:0042322], positive regulation of circadian sleep/wake cycle, REM sleep [GO:0046005] Also known as: regulation of REM sleep